{
  "term_label": "microtubule-based movement",
  "gene": "UniProtKB:Q8N7M0",
  "gene_name": "Dynein light chain Tctex-type 5",
  "gene_symbol": "DYNLT5",
  "term_id": "GO:0007018"
}